{
  "term_id": "GO:0098978",
  "gene_symbol": "DLGAP3",
  "term_label": "glutamatergic synapse",
  "gene": "UniProtKB:O95886",
  "gene_name": "Disks large-associated protein 3"
}